{
  "term_label": "endoplasmic reticulum",
  "gene_name": "Polyprenol reductase",
  "gene_symbol": "SRD5A3",
  "gene": "UniProtKB:Q9H8P0",
  "term_id": "GO:0005783"
}